{
  "term_id": "UNKNOWN:0003",
  "gene_name": "Putative uncharacterized protein encoded by LINC02915",
  "term_label": "Unknown cellular component",
  "gene_symbol": "LINC02915",
  "gene": "UniProtKB:Q8N8G6"
}